{
  "gene_symbol": "ZNF830",
  "gene_name": "Zinc finger protein 830",
  "term_id": "GO:0044773",
  "gene": "UniProtKB:Q96NB3",
  "term_label": "mitotic DNA damage checkpoint signaling"
}